{
  "gene_name": "Dual specificity protein phosphatase 6",
  "gene_symbol": "DUSP6",
  "gene": "UniProtKB:Q16828",
  "term_label": "regulation of heart growth",
  "term_id": "GO:0060420"
}